response to tamsulosin [GO:1901905] (BP) Definition: Any process that results in a change in state or activity of a cell or an organism (in terms of movement, secretion, enzyme production, gene expression, etc.) as a result of a tamsulosin stimulus. Sources: GOC:TermGenie Relationships: is a type of response to amine [GO:0014075]; is a type of response to ether [GO:0045472]